limonene catabolic process [GO:0046251] (biological process) Definition: The chemical reactions and pathways resulting in the breakdown of limonene (4-isopropenyl-1-methyl-cyclohexene), a monocyclic monoterpene. References: PMID:10224006 Also known as: limonene breakdown, limonene catabolism, limonene degradation Relationships: is a type of monoterpene catabolic process [GO:0043694]; is_a olefinic compound catabolic process [GO:0120256]; is a type of GO:1900673